K antigen biosynthetic process [GO:0009248] (biological process) Definition: The chemical reactions and pathways resulting in the formation of a K antigen, a capsular polysaccharide antigen carried on the surface of bacterial capsules that masks somatic (O) antigens. Relationships: is a type of GO:0000271; is a type of K antigen metabolic process [GO:0046375]; is a type of carbohydrate derivative biosynthetic process [GO:1901137] Also known as: K antigen anabolism, K antigen biosynthesis, K antigen formation, K antigen synthesis Sources: ISBN:0198506732